{
  "gene_symbol": "HSD17B6",
  "term_id": "GO:0042572",
  "gene": "UniProtKB:O14756",
  "gene_name": "17-beta-hydroxysteroid dehydrogenase type 6",
  "term_label": "retinol metabolic process"
}